{
  "term_label": "inward rectifier potassium channel activity",
  "gene": "UniProtKB:P48544",
  "gene_symbol": "KCNJ5",
  "gene_name": "G protein-activated inward rectifier potassium channel 4",
  "term_id": "GO:0005242"
}